{
  "gene_symbol": "KRTAP15-1",
  "gene": "UniProtKB:Q3LI76",
  "term_id": "UNKNOWN:0002",
  "term_label": "Unknown biological process",
  "gene_name": "Keratin-associated protein 15-1"
}